{
  "gene_symbol": "FOXA2",
  "gene_name": "Hepatocyte nuclear factor 3-beta",
  "term_id": "UNKNOWN:0003",
  "term_label": "Unknown cellular component",
  "gene": "UniProtKB:Q9Y261"
}